regulation of protein localization to endosome [GO:1905666] (biological process) Relationships: is a type of regulation of protein localization [GO:0032880]; regulates GO:0036010 Also known as: regulation of protein localisation in endosome, regulation of protein localization in endosome Subtypes: regulation of protein localization to early endosome [GO:1902965], negative regulation of protein localization to endosome [GO:1905667], positive regulation of protein localization to endosome [GO:1905668] References: PMID:22732145 Sources: GOC:PARL, GOC:TermGenie, GOC:bc, GO_REF:0000058 Definition: Any process that modulates the frequency, rate or extent of protein localization to endosome.